histone H2A ubiquitin ligase activity [GO:0141053] (molecular function) Relationships: is a type of histone ubiquitin ligase activity [GO:0140852] Subtypes: histone H2AK13 ubiquitin ligase activity [GO:0140856], histone H2AK15 ubiquitin ligase activity [GO:0140858], histone H2AK119 ubiquitin ligase activity [GO:0140862], histone H2AK127 ubiquitin ligase activity [GO:0140863], histone H2AK129 ubiquitin ligase activity [GO:0140864] References: PMID:25303536 Definition: Catalysis of the transfer of ubiquitin to a histone H2A substrate.